CMG complex [GO:0071162] (cellular component) Also known as: unwindosome References: PMID:19228417 Sources: GOC:rb Definition: A protein complex that contains the GINS complex, Cdc45p, and the heterohexameric MCM complex, and that is involved in unwinding DNA during replication. Relationships: is a type of DNA replication preinitiation complex [GO:0031261]; is part of nuclear chromosome [GO:0000228]; has part GINS complex [GO:0000811]